{
  "term_label": "complement activation, classical pathway",
  "gene": "UniProtKB:P01880",
  "gene_name": "Immunoglobulin heavy constant delta",
  "term_id": "GO:0006958",
  "gene_symbol": "IGHD"
}